{
  "gene_symbol": "TREM1",
  "term_id": "GO:0070945",
  "gene_name": "Triggering receptor expressed on myeloid cells 1",
  "term_label": "neutrophil-mediated killing of gram-negative bacterium",
  "gene": "UniProtKB:Q9NP99"
}